{
  "gene": "UniProtKB:Q9Y4Z0",
  "gene_name": "U6 snRNA-associated Sm-like protein LSm4",
  "term_label": "U6 snRNP",
  "term_id": "GO:0005688",
  "gene_symbol": "LSM4"
}